regulation of phospholipid biosynthetic process [GO:0071071] (biological process) Relationships: is a type of GO:0046890; is a type of regulation of phospholipid metabolic process [GO:1903725]; regulates phospholipid biosynthetic process [GO:0008654] Definition: Any process that modulates the frequency, rate or extent of the chemical reactions and pathways resulting in the formation of phospholipids. Sources: GOC:mah Also known as: regulation of phospholipid anabolism, regulation of phospholipid biosynthesis, regulation of phospholipid formation, regulation of phospholipid synthesis Subtypes: GO:0010322, regulation of phosphatidylinositol biosynthetic process [GO:0010511], regulation of dolichyl monophosphate biosynthetic process [GO:0010794], negative regulation of phospholipid biosynthetic process [GO:0071072], positive regulation of phospholipid biosynthetic process [GO:0071073], regulation of phosphatidylserine biosynthetic process [GO:1900468], regulation of phosphatidylglycerol biosynthetic process [GO:1901351], regulation of phosphatidic acid biosynthetic process [GO:1905693], regulation of isopentenyl diphosphate biosynthetic process, mevalonate pathway [GO:2001210], regulation of phosphatidylcholine biosynthetic process [GO:2001245]